inferior olivary nucleus maturation [GO:0021717] (biological process) Also known as: inferior olive maturation Relationships: is a type of anatomical structure maturation [GO:0071695]; is part of medulla oblongata maturation [GO:0021582]; is part of inferior olivary nucleus development [GO:0021713] Sources: GOC:cls, GOC:dgh, GOC:dph, GOC:jid, GO_REF:0000021 Definition: A developmental process, independent of morphogenetic (shape) change, that is required for the inferior olivary nucleus to attain its fully functional state. The inferior olivary nucleus is a capsule-shaped structure in the ventral medulla located just lateral and dorsal to the medullary pyramids. Neurons in the inferior olivary nucleus are the source of climbing fiber input to the cerebellar cortex; these neurons have been implicated in various functions, such as learning and timing of movements.